{
  "gene_symbol": "TMCO5A",
  "gene_name": "Transmembrane and coiled-coil domain-containing protein 5A",
  "gene": "UniProtKB:Q8N6Q1",
  "term_id": "UNKNOWN:0002",
  "term_label": "Unknown biological process"
}